glucuronokinase activity [GO:0047940] (molecular function) Definition: Catalysis of the reaction: D-glucuronate + ATP = 1-phospho-alpha-D-glucuronate + ADP + 2 H+. Sources: EC:2.7.1.43, RHEA:17005 Also known as: ATP:D-glucuronate 1-phosphotransferase activity, glucurono-glucuronokinase activity, glucuronokinase (phosphorylating) Relationships: is a type of kinase activity [GO:0016301]; is a type of phosphotransferase activity, alcohol group as acceptor [GO:0016773]